positive regulation of response to DNA integrity checkpoint signaling [GO:1902152] (biological process) Relationships: is a type of positive regulation of response to cell cycle checkpoint signaling [GO:1902146]; is a type of regulation of response to DNA integrity checkpoint signaling [GO:1902151]; positively regulates response to DNA integrity checkpoint signaling [GO:0072402] Also known as: activation of DNA integrity checkpoint effector process, activation of response to signal involved in DNA integrity checkpoint, positive regulation of DNA integrity checkpoint effector process, positive regulation of response to signal involved in DNA integrity checkpoint, up regulation of DNA integrity checkpoint effector process, up regulation of response to DNA integrity checkpoint signaling, up regulation of response to signal involved in DNA integrity checkpoint, up-regulation of DNA integrity checkpoint effector process, up-regulation of response to DNA integrity checkpoint signaling, up-regulation of response to signal involved in DNA integrity checkpoint, upregulation of DNA integrity checkpoint effector process, upregulation of response to DNA integrity checkpoint signaling, upregulation of response to signal involved in DNA integrity checkpoint, activation of response to DNA integrity checkpoint signaling Subtypes: GO:1902154 Definition: Any process that activates or increases the frequency, rate or extent of response to DNA integrity checkpoint signaling. Sources: GOC:TermGenie, GOC:mtg_cell_cycle